{
  "term_id": "GO:0007224",
  "gene_symbol": "STK36",
  "gene": "UniProtKB:Q9NRP7",
  "gene_name": "Serine_threonine-protein kinase 36",
  "term_label": "smoothened signaling pathway"
}